{
  "gene": "UniProtKB:Q08345",
  "term_label": "positive regulation of phosphatidylinositol 3-kinase/protein kinase B signal transduction",
  "gene_symbol": "DDR1",
  "gene_name": "Epithelial discoidin domain-containing receptor 1",
  "term_id": "GO:0051897"
}